negative regulation of snoRNA processing [GO:1902797] (biological process) Definition: Any process that stops, prevents or reduces the frequency, rate or extent of snoRNA processing. Relationships: is a type of GO:0010629; is a type of GO:1902796; is a type of negative regulation of snoRNA metabolic process [GO:1903324]; negatively regulates sno(s)RNA processing [GO:0043144] Also known as: down regulation of snoRNA processing, down-regulation of snoRNA processing, downregulation of snoRNA processing, inhibition of snoRNA processing References: PMID:24210919 Sources: GOC:TermGenie, GO_REF:0000058